{
  "term_id": "GO:0051015",
  "gene": "UniProtKB:O75146",
  "gene_name": "Huntingtin-interacting protein 1-related protein",
  "term_label": "actin filament binding",
  "gene_symbol": "HIP1R"
}